{
  "gene_symbol": "MTOR",
  "term_id": "GO:0004674",
  "term_label": "protein serine/threonine kinase activity",
  "gene_name": "Serine_threonine-protein kinase mTOR",
  "gene": "UniProtKB:P42345"
}